{
  "gene": "UniProtKB:Q86UF2",
  "gene_symbol": "CTAGE6",
  "gene_name": "cTAGE family member 6",
  "term_label": "endoplasmic reticulum to Golgi vesicle-mediated transport",
  "term_id": "GO:0006888"
}